{
  "gene_symbol": "KLHL12",
  "gene_name": "Kelch-like protein 12",
  "term_id": "GO:0043161",
  "gene": "UniProtKB:Q53G59",
  "term_label": "proteasome-mediated ubiquitin-dependent protein catabolic process"
}